{
  "term_id": "GO:0051901",
  "gene": "UniProtKB:Q13015",
  "term_label": "positive regulation of mitochondrial depolarization",
  "gene_symbol": "MLLT11",
  "gene_name": "Protein AF1q"
}